{
  "gene_name": "tRNA (cytosine(38)-C(5))-methyltransferase",
  "gene_symbol": "TRDMT1",
  "term_label": "tRNA (cytidine-5-)-methyltransferase activity",
  "gene": "UniProtKB:O14717",
  "term_id": "GO:0016428"
}